{
  "gene": "UniProtKB:Q9NPF5",
  "gene_name": "DNA methyltransferase 1-associated protein 1",
  "term_label": "NuA4 histone acetyltransferase complex",
  "term_id": "GO:0035267",
  "gene_symbol": "DMAP1"
}